{
  "gene_name": "Transmembrane protein 176B",
  "term_id": "UNKNOWN:0003",
  "gene": "UniProtKB:Q3YBM2",
  "term_label": "Unknown cellular component",
  "gene_symbol": "TMEM176B"
}